{
  "gene_name": "Sodium channel subunit beta-1",
  "term_label": "sodium channel inhibitor activity",
  "gene_symbol": "SCN1B",
  "gene": "UniProtKB:Q07699",
  "term_id": "GO:0019871"
}